{
  "gene_name": "Protein FAM110A",
  "gene_symbol": "FAM110A",
  "gene": "UniProtKB:Q9BQ89",
  "term_id": "UNKNOWN:0002",
  "term_label": "Unknown biological process"
}